{
  "term_id": "GO:0005886",
  "gene": "UniProtKB:Q4VCS5",
  "gene_name": "Angiomotin",
  "gene_symbol": "AMOT",
  "term_label": "plasma membrane"
}